{
  "term_id": "GO:0005654",
  "term_label": "nucleoplasm",
  "gene": "UniProtKB:Q6IEG0",
  "gene_symbol": "SNRNP48",
  "gene_name": "U11_U12 small nuclear ribonucleoprotein 48 kDa protein"
}